bone growth [GO:0098868] (biological process) Definition: The increase in size or mass of a bone that contributes to the shaping of that bone. Relationships: is a type of organ growth [GO:0035265]; is part of bone development [GO:0060348] Sources: GOC:dos Subtypes: endochondral bone growth [GO:0003416], intramembranous bone growth [GO:0098867]